membrane bending activity [GO:0180020] (MF) Definition: The activity of bending or deforming a membrane. This activity can occur by multiple mechanisms including the insertion amphipathic domains into one or both leaflets. References: PMID:19780639 Also known as: membrane curving Relationships: is a type of GO:0003674